{
  "gene_name": "Alpha-1,6-mannosylglycoprotein 6-beta-N-acetylglucosaminyltransferase B",
  "term_label": "alpha-1,6-mannosylglycoprotein 6-beta-N-acetylglucosaminyltransferase activity",
  "gene": "UniProtKB:Q3V5L5",
  "term_id": "GO:0030144",
  "gene_symbol": "MGAT5B"
}